{
  "gene": "UniProtKB:Q96DZ7",
  "term_id": "GO:0016020",
  "gene_symbol": "TM4SF19",
  "term_label": "membrane",
  "gene_name": "Transmembrane 4 L6 family member 19"
}